{
  "gene_symbol": "NUTM1",
  "gene": "UniProtKB:Q86Y26",
  "term_label": "Unknown biological process",
  "gene_name": "NUT family member 1",
  "term_id": "UNKNOWN:0002"
}